{
  "gene": "UniProtKB:Q7Z3J3",
  "term_id": "GO:0051168",
  "gene_name": "RanBP2-like and GRIP domain-containing protein 4",
  "term_label": "nuclear export",
  "gene_symbol": "RGPD4"
}